{
  "term_label": "GDP phosphatase activity",
  "term_id": "GO:0004382",
  "gene": "UniProtKB:Q9Y5L3",
  "gene_symbol": "ENTPD2",
  "gene_name": "Ectonucleoside triphosphate diphosphohydrolase 2"
}